muscle cell proliferation [GO:0033002] (biological process) Also known as: myocyte proliferation Relationships: is a type of GO:0008283 Sources: CL:0000187, GOC:mah Subtypes: GO:0014855, GO:0048659 Definition: The expansion of a muscle cell population by cell division.